{
  "gene": "UniProtKB:Q8IYU8",
  "gene_name": "Calcium uptake protein 2, mitochondrial",
  "gene_symbol": "MICU2",
  "term_label": "uniplex complex",
  "term_id": "GO:1990246"
}